ubiquinone catabolic process [GO:0032322] (biological process) Also known as: ubiquinone breakdown, ubiquinone catabolism, ubiquinone degradation Sources: GOC:mah Definition: The chemical reactions and pathways resulting in the breakdown of ubiquinone, a lipid-soluble electron-transporting coenzyme. Relationships: is_a ubiquinone metabolic process [GO:0006743]; is_a quinone catabolic process [GO:1901662]